{
  "term_id": "GO:0015986",
  "gene": "UniProtKB:P05496",
  "gene_name": "ATP synthase F(0) complex subunit C1, mitochondrial",
  "gene_symbol": "ATP5MC1",
  "term_label": "proton motive force-driven ATP synthesis"
}